modulation of formation of symbiont germ tube hook structure for appressorium development [GO:0075030] (biological process) Definition: Any process that modulates the frequency, rate or extent of symbiont germ tube hook structure formation. Subtypes: positive regulation of formation of symbiont germ tube hook structure for appressorium development [GO:0075031], negative regulation of formation of symbiont germ tube hook structure for appressorium development [GO:0075032] Relationships: is_a GO:0050793; regulates formation of appressorium germ tube hook structure [GO:0075029] Also known as: modulation of germ tube tip of symbiont on or near the exterior of host, regulation of formation of symbiont germ tube hook structure on or near host, modulation of symbiont germ tube hook structure formation on or near host Sources: GOC:pamgo_curators